{
  "gene_symbol": "NUP155",
  "term_label": "transcription-dependent tethering of RNA polymerase II gene DNA at nuclear periphery",
  "term_id": "GO:0000972",
  "gene_name": "Nuclear pore complex protein Nup155",
  "gene": "UniProtKB:O75694"
}